{
  "gene_name": "Ferritin heavy chain",
  "term_id": "GO:0005737",
  "gene_symbol": "FTH1",
  "term_label": "cytoplasm",
  "gene": "UniProtKB:P02794"
}